positive regulation of cytokine production involved in inflammatory response [GO:1900017] (BP) Also known as: up regulation of cytokine production involved in acute inflammatory response, positive regulation of cytokine production involved in acute inflammatory response, up regulation of cytokine production involved in inflammatory response Sources: GOC:TermGenie Definition: Any process that activates or increases the frequency, rate or extent of cytokine production involved in inflammatory response. Relationships: is a type of positive regulation of cytokine production [GO:0001819]; is a type of regulation of cytokine production involved in inflammatory response [GO:1900015]; positively regulates cytokine production involved in inflammatory response [GO:0002534]